{
  "gene": "UniProtKB:O75712",
  "term_id": "GO:0005922",
  "term_label": "connexin complex",
  "gene_name": "Gap junction beta-3 protein",
  "gene_symbol": "GJB3"
}